cyclin D3-CDK4 complex [GO:0097130] (cellular component) Definition: A protein complex consisting of cyclin D3 and cyclin-dependent kinase 4 (CDK4). Cyclins are characterized by periodicity in protein abundance throughout the cell cycle. Cyclin-dependent kinases represent a family of serine/threonine protein kinases that become active upon binding to a cyclin regulatory partner. References: PMID:15935619 Sources: GOC:so Relationships: is a type of cyclin-dependent protein kinase holoenzyme complex [GO:0000307]